4-chlorobenzoate dehalogenase activity [GO:0047576] (molecular function) Definition: Catalysis of the reaction: 4-chlorobenzoate + H2O = 4-hydroxybenzoate + chloride + H+. Sources: RHEA:23440 Also known as: 4-chlorobenzoate chlorohydrolase activity, halobenzoate dehalogenase activity Relationships: is a type of GO:0019120